{
  "gene": "UniProtKB:Q03721",
  "term_label": "presynaptic membrane",
  "gene_symbol": "KCNC4",
  "term_id": "GO:0042734",
  "gene_name": "Potassium voltage-gated channel subfamily C member 4"
}